{
  "gene_symbol": "HLA-DPA1",
  "gene_name": "HLA class II histocompatibility antigen, DP alpha 1 chain",
  "term_id": "GO:0042605",
  "term_label": "peptide antigen binding",
  "gene": "UniProtKB:P20036"
}